{
  "term_id": "GO:0006516",
  "gene_name": "F-box only protein 6",
  "gene_symbol": "FBXO6",
  "gene": "UniProtKB:Q9NRD1",
  "term_label": "glycoprotein catabolic process"
}